{
  "term_label": "Golgi apparatus",
  "gene_name": "Transmembrane emp24 domain-containing protein 3",
  "gene": "UniProtKB:Q9Y3Q3",
  "gene_symbol": "TMED3",
  "term_id": "GO:0005794"
}